{
  "gene_symbol": "TRDJ2",
  "gene_name": "T cell receptor delta joining 2 (Fragment)",
  "gene": "UniProtKB:A0A075B6V6",
  "term_id": "UNKNOWN:0002",
  "term_label": "Unknown biological process"
}